{
  "gene_symbol": "ZNF135",
  "term_id": "GO:0005634",
  "gene": "UniProtKB:P52742",
  "term_label": "nucleus",
  "gene_name": "Zinc finger protein 135"
}